R-lactaldehyde reductase activity [GO:0052660] (molecular function) Also known as: (R)-propane-1,2-diol:NAD+ oxidoreductase activity, D-lactaldehyde:propanediol oxidoreductase activity Sources: RHEA:23872 Definition: Catalysis of the reaction: (R)-propane-1,2-diol + NAD+ = (R)-lactaldehyde + NADH + H+. Relationships: is a type of lactaldehyde reductase activity [GO:0008912]